serotonin-activated cation-selective channel complex [GO:1904602] (cellular component) Note: An example of this is HTR3A in human (P46098) in PMID:16116092 (inferred from direct assay). References: PMID:16116092 Sources: GOC:TermGenie, GOC:bhm, GO_REF:0000088 Relationships: is a type of GO:0034703; is a type of serotonin receptor complex [GO:0098665]; is a type of GO:0098878 Also known as: serotonin receptor complex, 5-HT-3 receptor complex, 5-HT3 receptor complex, 5-hydroxytryptamine receptor 3 complex, 5HT3 receptor complex Definition: A protein complex which is capable of serotonin-activated cation-selective channel activity. Mainly found in pre- and postsynaptic membranes of the brain and gastrointestinal tract. Depending on its location it transports Ca2+, Mg2+, Na+ or K+. It is always a pentamer, containing at least the 5HT3A subunit forming 5HT3A homopentamers or 5HT3A/B heteropentamers. In human, 5HT3A/C, A/D and A/E heteropentamers also exist.